positive regulation of thyroid hormone generation [GO:2000611] (biological process) Sources: GOC:obol Relationships: is a type of positive regulation of hormone metabolic process [GO:0032352]; is a type of regulation of thyroid hormone generation [GO:2000609]; positively regulates thyroid hormone generation [GO:0006590] Definition: Any process that activates or increases the frequency, rate or extent of thyroid hormone generation.